negative regulation of interleukin-3 production [GO:0032712] (biological process) Sources: GOC:mah Relationships: is a type of negative regulation of cytokine production [GO:0001818]; is a type of regulation of interleukin-3 production [GO:0032672]; negatively regulates interleukin-3 production [GO:0032632] Also known as: down regulation of interleukin-3 production, down-regulation of interleukin-3 production, downregulation of interleukin-3 production, negative regulation of IL-3 production, inhibition of interleukin-3 production, negative regulation of interleukin-3 biosynthetic process Definition: Any process that stops, prevents, or reduces the frequency, rate, or extent of interleukin-3 production.